{
  "gene_name": "Adhesion G protein-coupled receptor A3",
  "gene": "UniProtKB:Q8IWK6",
  "gene_symbol": "ADGRA3",
  "term_label": "plasma membrane",
  "term_id": "GO:0005886"
}